exodeoxyribonuclease VII activity [GO:0008855] (molecular function) Definition: Catalysis of the exonucleolytic cleavage in either 5' to 3' or 3' to 5' direction to yield 5'-phosphomononucleotides. Sources: EC:3.1.11.6 Also known as: E. coli exonuclease VII activity, E. coli exonuclease VII, Escherichia coli exonuclease VII, endodeoxyribonuclease VII, exonuclease VII activity Relationships: is a type of GO:0016895